{
  "term_id": "UNKNOWN:0003",
  "term_label": "Unknown cellular component",
  "gene_name": "Zinc finger protein 675",
  "gene_symbol": "ZNF675",
  "gene": "UniProtKB:Q8TD23"
}